{
  "gene": "UniProtKB:Q96M78",
  "gene_symbol": "FER1L6-AS2",
  "gene_name": "Putative uncharacterized protein encoded by FER1L6-AS2",
  "term_id": "UNKNOWN:0001",
  "term_label": "Unknown molecular function"
}